regulation of vesicle-mediated transport [GO:0060627] (biological process) Definition: Any process that modulates the rate, frequency, or extent of vesicle-mediated transport, the directed movement of substances, either within a vesicle or in the vesicle membrane, into, out of or within a cell. Subtypes: regulation of exocytosis [GO:0017157], regulation of endocytosis [GO:0030100], regulation of vesicle fusion [GO:0031338], GO:0042996, regulation of ER to Golgi vesicle-mediated transport [GO:0060628], regulation of synaptic vesicle cycle [GO:0098693], regulation of early endosome to recycling endosome transport [GO:1902954], GO:1904298, regulation of retrograde transport, endosome to Golgi [GO:1905279], regulation of retrograde vesicle-mediated transport, Golgi to ER [GO:2000156], regulation of early endosome to late endosome transport [GO:2000641], regulation of endocytic recycling [GO:2001135] Relationships: is a type of GO:0050794; is a type of GO:0051049; regulates GO:0016192 Sources: GOC:dph, GOC:tb